{
  "gene_symbol": "PGF",
  "term_id": "GO:0048010",
  "gene": "UniProtKB:P49763",
  "term_label": "vascular endothelial growth factor receptor signaling pathway",
  "gene_name": "Placenta growth factor"
}